{
  "gene": "UniProtKB:Q8NGS3",
  "term_label": "plasma membrane",
  "term_id": "GO:0005886",
  "gene_symbol": "OR1J1",
  "gene_name": "Olfactory receptor 1J1"
}